{
  "gene_symbol": "MEIS2",
  "gene_name": "Homeobox protein Meis2",
  "term_label": "positive regulation of transcription by RNA polymerase II",
  "term_id": "GO:0045944",
  "gene": "UniProtKB:O14770"
}